regulation of chitin-based cuticle tanning [GO:0007564] (biological process) Definition: Any process that modulates the frequency, rate or extent of chitin-based cuticular tanning. Sources: GOC:go_curators, GOC:jid, GOC:mtg_sensu Relationships: is a type of regulation of multicellular organismal development [GO:2000026]; regulates chitin-based cuticle sclerotization [GO:0007593] Also known as: regulation of cuticle tanning, regulation of cuticle hardening Subtypes: negative regulation of chitin-based cuticle tanning [GO:0045800], GO:0045801